{
  "term_label": "nucleus",
  "term_id": "GO:0005634",
  "gene_symbol": "NMD3",
  "gene_name": "60S ribosomal export protein NMD3",
  "gene": "UniProtKB:Q96D46"
}